negative regulation of transforming growth factor beta2 production [GO:0032912] (biological process) Also known as: down regulation of transforming growth factor-beta2 production, down-regulation of transforming growth factor-beta2 production, downregulation of transforming growth factor-beta2 production, negative regulation of TGF-B2 production, negative regulation of TGFB2 production, negative regulation of transforming growth factor-beta2 production, inhibition of transforming growth factor-beta2 production Definition: Any process that stops, prevents, or reduces the frequency, rate, or extent of production of transforming growth factor-beta2. Sources: GOC:mah Relationships: is a type of GO:0032909; is a type of negative regulation of transforming growth factor beta production [GO:0071635]; negatively regulates transforming growth factor beta2 production [GO:0032906]